{
  "gene_name": "Protein TAMALIN",
  "term_id": "GO:0007165",
  "gene_symbol": "TAMALIN",
  "term_label": "signal transduction",
  "gene": "UniProtKB:Q7Z6J2"
}